{
  "term_id": "GO:0031594",
  "gene_symbol": "DLG3",
  "gene": "UniProtKB:Q92796",
  "gene_name": "Disks large homolog 3",
  "term_label": "neuromuscular junction"
}